histamine metabolic process [GO:0001692] (biological process) Subtypes: histamine biosynthetic process [GO:0001694], histamine catabolic process [GO:0001695] Sources: GOC:jl, ISBN:0395825172 Relationships: is a type of biogenic amine metabolic process [GO:0006576]; is a type of imidazole-containing compound metabolic process [GO:0052803] Definition: The chemical reactions and pathways involving histamine, a physiologically active amine, found in plant and animal tissue and released from mast cells as part of an allergic reaction in humans. Also known as: histamine metabolism